{
  "gene": "UniProtKB:Q8NA72",
  "gene_symbol": "POC5",
  "term_label": "eye photoreceptor cell development",
  "gene_name": "Centrosomal protein POC5",
  "term_id": "GO:0042462"
}